{
  "gene_name": "Large ribosomal subunit protein uL13",
  "term_label": "mRNA binding",
  "term_id": "GO:0003729",
  "gene": "UniProtKB:P40429",
  "gene_symbol": "RPL13A"
}